{
  "gene": "UniProtKB:Q147X3",
  "gene_symbol": "NAA30",
  "gene_name": "N-alpha-acetyltransferase 30",
  "term_id": "GO:0031417",
  "term_label": "NatC complex"
}